{
  "gene_symbol": "HAPSTR1",
  "term_id": "UNKNOWN:0002",
  "gene_name": "HUWE1-associated protein modifying stress responses 1",
  "gene": "UniProtKB:Q14CZ0",
  "term_label": "Unknown biological process"
}